{
  "gene": "UniProtKB:Q8TD86",
  "term_id": "GO:0030234",
  "term_label": "enzyme regulator activity",
  "gene_name": "Calmodulin-like protein 6",
  "gene_symbol": "CALML6"
}